{
  "term_id": "GO:0044224",
  "gene_name": "Voltage-gated potassium channel subunit beta-2",
  "gene_symbol": "KCNAB2",
  "term_label": "juxtaparanode region of axon",
  "gene": "UniProtKB:Q13303"
}